androecium development [GO:0048466] (biological process) Definition: The process whose specific outcome is the progression of the androecium over time, from its formation to the mature structure. Relationships: is a type of floral whorl development [GO:0048438] Sources: GOC:go_curators